excinuclease repair complex [GO:0009380] (cellular component) References: PMID:12145219, PMID:15192705 Sources: GOC:mah, GOC:mlg Also known as: UvrABC excinuclease complex, excinuclease ABC complex Definition: Any of the protein complexes formed by the UvrABC excinuclease system, which carries out nucleotide excision repair. Three different complexes are formed by the 3 proteins as they proceed through the excision repair process. First a complex consisting of two A subunits and two B subunits bind DNA and unwind it around the damaged site. Then, the A subunits disassociate leaving behind a stable complex between B subunits and DNA. Now, subunit C binds to this B+DNA complex and causes subunit B to nick the DNA on one side of the complex while subunit C nicks the DNA on the other side of the complex. DNA polymerase I and DNA ligase can then repair the resulting gap. Relationships: is_a GO:1905347; is a type of DNA repair complex [GO:1990391]